{
  "gene_symbol": "CEACAM20",
  "term_id": "GO:0007165",
  "gene": "UniProtKB:Q6UY09",
  "gene_name": "Carcinoembryonic antigen-related cell adhesion molecule 20",
  "term_label": "signal transduction"
}